{
  "gene": "UniProtKB:Q8N7Y1",
  "gene_symbol": "KIRREL3-AS3",
  "term_id": "UNKNOWN:0002",
  "term_label": "Unknown biological process",
  "gene_name": "Putative uncharacterized protein KIRREL3-AS3"
}